{
  "term_label": "cytoplasm",
  "gene_name": "Leucine-rich repeat-containing protein 75A",
  "term_id": "GO:0005737",
  "gene_symbol": "LRRC75A",
  "gene": "UniProtKB:Q8NAA5"
}